{
  "term_label": "ATPase binding",
  "term_id": "GO:0051117",
  "gene": "UniProtKB:Q93050",
  "gene_name": "V-type proton ATPase 116 kDa subunit a 1",
  "gene_symbol": "ATP6V0A1"
}